{
  "term_id": "GO:0005634",
  "gene": "UniProtKB:Q13315",
  "gene_symbol": "ATM",
  "term_label": "nucleus",
  "gene_name": "Serine-protein kinase ATM"
}